{
  "gene_name": "SPRY domain-containing SOCS box protein 1",
  "term_id": "GO:0043161",
  "gene": "UniProtKB:Q96BD6",
  "term_label": "proteasome-mediated ubiquitin-dependent protein catabolic process",
  "gene_symbol": "SPSB1"
}